{
  "term_label": "ubiquitin-like ligase-substrate adaptor activity",
  "term_id": "GO:1990756",
  "gene_name": "Protein fem-1 homolog A",
  "gene_symbol": "FEM1A",
  "gene": "UniProtKB:Q9BSK4"
}